{
  "gene_name": "Staphylococcal nuclease domain-containing protein 1",
  "gene": "UniProtKB:Q7KZF4",
  "gene_symbol": "SND1",
  "term_id": "GO:0005829",
  "term_label": "cytosol"
}